{
  "term_id": "UNKNOWN:0003",
  "gene_symbol": "OR8U9",
  "gene_name": "Olfactory receptor 8U9",
  "gene": "UniProtKB:P0C7N5",
  "term_label": "Unknown cellular component"
}